{
  "gene": "UniProtKB:Q96PP4",
  "gene_name": "Testis-specific gene 13 protein",
  "term_id": "UNKNOWN:0002",
  "term_label": "Unknown biological process",
  "gene_symbol": "TSGA13"
}